maintenance of right sidedness [GO:0061970] (biological process) Definition: The organization process that preserves the right sidedness in an organism's body plan or part of an organism with respect to the left and right halves. References: PMID:18629866 Sources: GOC:BHF Relationships: is a type of GO:0061968